regulation of tyrosine phosphorylation of STAT protein [GO:0042509] (biological process) Subtypes: positive regulation of tyrosine phosphorylation of STAT protein [GO:0042531], negative regulation of tyrosine phosphorylation of STAT protein [GO:0042532] References: PMID:11426647 Sources: GOC:jl Definition: Any process that modulates the frequency, rate or extent of the introduction of a phosphate group to a tyrosine residue of a STAT (Signal Transducer and Activator of Transcription) protein. Relationships: is a type of regulation of peptidyl-tyrosine phosphorylation [GO:0050730]; regulates tyrosine phosphorylation of STAT protein [GO:0007260] Also known as: regulation of tyrosine phosphorylation of Stat1 protein, regulation of tyrosine phosphorylation of Stat2 protein, regulation of tyrosine phosphorylation of Stat3 protein, regulation of tyrosine phosphorylation of Stat4 protein, regulation of tyrosine phosphorylation of Stat5 protein, regulation of tyrosine phosphorylation of Stat6 protein, regulation of tyrosine phosphorylation of Stat7 protein